{
  "gene": "UniProtKB:Q2VIR3",
  "gene_symbol": "EIF2S3B",
  "gene_name": "Eukaryotic translation initiation factor 2 subunit 3B",
  "term_label": "eukaryotic translation initiation factor 2 complex",
  "term_id": "GO:0005850"
}